{
  "gene_name": "Phospholipid phosphatase-related protein type 2",
  "gene": "UniProtKB:Q96GM1",
  "gene_symbol": "PLPPR2",
  "term_id": "GO:0008195",
  "term_label": "phosphatidate phosphatase activity"
}